{
  "gene_symbol": "PLK3",
  "term_id": "GO:0004674",
  "gene": "UniProtKB:Q9H4B4",
  "term_label": "protein serine/threonine kinase activity",
  "gene_name": "Serine_threonine-protein kinase PLK3"
}